phospholipid dephosphorylation [GO:0046839] (biological process) Subtypes: GO:0046856 Sources: ISBN:0198506732 Relationships: is a type of GO:0016311; is a type of lipid modification [GO:0030258] Definition: The process of removing one or more phosphate groups from a phosphorylated lipid, any member of a group of substances soluble in lipid solvents but only sparingly soluble in aqueous solvents.